{
  "term_label": "negative regulation of transcription by RNA polymerase II",
  "term_id": "GO:0000122",
  "gene_symbol": "MAGEA1",
  "gene_name": "Melanoma-associated antigen 1",
  "gene": "UniProtKB:P43355"
}